{
  "gene_symbol": "SHROOM4",
  "term_id": "GO:0030864",
  "gene": "UniProtKB:Q9ULL8",
  "gene_name": "Protein Shroom4",
  "term_label": "cortical actin cytoskeleton"
}